{
  "term_label": "Unknown cellular component",
  "gene": "UniProtKB:Q6PL24",
  "term_id": "UNKNOWN:0003",
  "gene_symbol": "TMED8",
  "gene_name": "Protein TMED8"
}